{
  "term_label": "regulation of DNA-templated transcription",
  "gene_symbol": "NAB1",
  "term_id": "GO:0006355",
  "gene": "UniProtKB:Q13506",
  "gene_name": "NGFI-A-binding protein 1"
}